{
  "term_id": "GO:0005739",
  "gene": "UniProtKB:Q6ZT89",
  "gene_symbol": "SLC25A48",
  "term_label": "mitochondrion",
  "gene_name": "Solute carrier family 25 member 48"
}